{
  "term_id": "GO:0000981",
  "gene_symbol": "NR4A1",
  "gene": "UniProtKB:P22736",
  "gene_name": "Nuclear receptor subfamily 4 group A member 1",
  "term_label": "DNA-binding transcription factor activity, RNA polymerase II-specific"
}